{
  "gene_name": "Probable non-functional T cell receptor beta variable 17",
  "gene": "UniProtKB:A0A087X0K7",
  "gene_symbol": "TRBV17",
  "term_label": "Unknown molecular function",
  "term_id": "UNKNOWN:0001"
}